regulation of oxidative stress-induced neuron intrinsic apoptotic signaling pathway [GO:1903376] (biological process) Sources: GOC:PARL, GOC:TermGenie, GOC:bf, GO_REF:0000058 Definition: Any process that modulates the frequency, rate or extent of oxidative stress-induced neuron intrinsic apoptotic signaling pathway. Subtypes: negative regulation of oxidative stress-induced neuron intrinsic apoptotic signaling pathway [GO:1903377], positive regulation of oxidative stress-induced neuron intrinsic apoptotic signaling pathway [GO:1903378], regulation of hydrogen peroxide-induced neuron intrinsic apoptotic signaling pathway [GO:1903383] Relationships: is_a regulation of neuron apoptotic process [GO:0043523]; is a type of GO:1902175; regulates GO:0036480 Also known as: regulation of oxidative stress-induced neuron apoptosis, regulation of oxidative stress-induced neuronal apoptosis, regulation of neuron intrinsic apoptotic signaling pathway in response to oxidative stress, regulation of neuron apoptosis in response to oxidative stress